{
  "gene_name": "Immunoglobulin kappa variable 1D-12",
  "gene": "UniProtKB:P01611",
  "term_label": "immunoglobulin complex",
  "gene_symbol": "IGKV1D-12",
  "term_id": "GO:0019814"
}